{
  "gene": "UniProtKB:O75467",
  "term_id": "GO:0000981",
  "gene_name": "Zinc finger protein 324A",
  "term_label": "DNA-binding transcription factor activity, RNA polymerase II-specific",
  "gene_symbol": "ZNF324"
}